{
  "gene_name": "G-protein coupled receptor 26",
  "gene_symbol": "GPR26",
  "term_id": "GO:0007189",
  "term_label": "adenylate cyclase-activating G protein-coupled receptor signaling pathway",
  "gene": "UniProtKB:Q8NDV2"
}